{
  "gene_name": "Rab GTPase-activating protein 1-like",
  "term_label": "Unknown cellular component",
  "gene_symbol": "RABGAP1L",
  "gene": "UniProtKB:Q5R372",
  "term_id": "UNKNOWN:0003"
}